complement component C1q complex [GO:0062167] (cellular component) Definition: A protein-containing complex composed of six subunits of each of the three homologous polypeptide chains C1QA, C1QB, and C1QB. It is a subunit of the complement C1 complex. In addition to complement activation, C1q appears to have roles in homeostasis and cellular development, superoxide (O2-) production by neutrophils, blood coagulation and neurological synapse pruning. Also known as: C1q, Complement 1q References: PMID:29449492 Relationships: is a type of protein-containing complex [GO:0032991]; is part of GO:0005576